{
  "term_id": "UNKNOWN:0002",
  "gene_symbol": "SCYGR4",
  "term_label": "Unknown biological process",
  "gene_name": "Small cysteine and glycine repeat-containing protein 4",
  "gene": "UniProtKB:A0A286YEV6"
}